{
  "term_label": "cytoplasmic microtubule organization",
  "gene": "UniProtKB:Q96RT8",
  "gene_symbol": "TUBGCP5",
  "gene_name": "Gamma-tubulin complex component 5",
  "term_id": "GO:0031122"
}